{
  "gene": "UniProtKB:P13500",
  "term_label": "positive regulation of cell migration",
  "term_id": "GO:0030335",
  "gene_symbol": "CCL2",
  "gene_name": "C-C motif chemokine 2"
}